{
  "gene_name": "Protein FAM153A",
  "term_id": "UNKNOWN:0001",
  "term_label": "Unknown molecular function",
  "gene_symbol": "FAM153A",
  "gene": "UniProtKB:Q9UHL3"
}